{
  "gene": "UniProtKB:Q96LD1",
  "gene_symbol": "SGCZ",
  "term_id": "GO:0042383",
  "gene_name": "Zeta-sarcoglycan",
  "term_label": "sarcolemma"
}